90S preribosome [GO:0030686] (cellular component) References: PMID:12150911, PMID:12957375, PMID:15120992 Sources: GOC:krc, GOC:vw Relationships: is a type of preribosome [GO:0030684]; has part t-UTP complex [GO:0034455] Definition: A large ribonucleoprotein complex considered to be the earliest preribosomal complex. In S. cerevisiae, it has a size of 90S and consists of the 35S pre-rRNA, early-associating ribosomal proteins most of which are part of the small ribosomal subunit, the U3 snoRNA and associated proteins.